{
  "term_label": "polyamine transmembrane transport",
  "gene_name": "Probable cation-transporting ATPase 13A4",
  "term_id": "GO:1902047",
  "gene_symbol": "ATP13A4",
  "gene": "UniProtKB:Q4VNC1"
}